{
  "gene_name": "Kinesin-like protein KIFC1",
  "gene": "UniProtKB:Q9BW19",
  "term_label": "nucleus",
  "term_id": "GO:0005634",
  "gene_symbol": "KIFC1"
}